{
  "gene_symbol": "CSNK1E",
  "term_id": "GO:0005737",
  "gene_name": "Casein kinase I isoform epsilon",
  "term_label": "cytoplasm",
  "gene": "UniProtKB:P49674"
}